{
  "gene": "UniProtKB:Q8NGQ3",
  "gene_name": "Olfactory receptor 1S2",
  "gene_symbol": "OR1S2",
  "term_label": "plasma membrane",
  "term_id": "GO:0005886"
}